{
  "gene_name": "T cell receptor alpha variable 8-4",
  "gene_symbol": "TRAV8-4",
  "term_id": "GO:0002250",
  "term_label": "adaptive immune response",
  "gene": "UniProtKB:P01737"
}